{
  "gene_name": "Vitronectin",
  "gene": "UniProtKB:P04004",
  "term_label": "integrin binding",
  "term_id": "GO:0005178",
  "gene_symbol": "VTN"
}